osteoclast maturation [GO:0036179] (biological process) Sources: CL:0000092, GOC:pg Also known as: chondroclast maturation Relationships: is a type of cell maturation [GO:0048469]; is part of osteoclast development [GO:0036035] Definition: A developmental process, independent of morphogenetic (shape) change, that is required for an osteoclast cell to attain its fully functional state. An osteoclast is a specialized phagocytic cell associated with the absorption and removal of the mineralized matrix of bone tissue, and which typically differentiates from monocytes.